{
  "gene_name": "Peroxisomal 2,4-dienoyl-CoA reductase [(3E)-enoyl-CoA-producing]",
  "term_id": "GO:0006631",
  "term_label": "fatty acid metabolic process",
  "gene": "UniProtKB:Q9NUI1",
  "gene_symbol": "DECR2"
}